regulation of fat cell differentiation [GO:0045598] (biological process) Sources: GOC:go_curators Subtypes: GO:0045599, positive regulation of fat cell differentiation [GO:0045600], regulation of brown fat cell differentiation [GO:0090335] Relationships: is a type of regulation of cell differentiation [GO:0045595]; regulates fat cell differentiation [GO:0045444] Definition: Any process that modulates the frequency, rate or extent of adipocyte differentiation. Also known as: regulation of adipocyte cell differentiation, regulation of adipocyte differentiation